{
  "gene_name": "TYRO protein tyrosine kinase-binding protein",
  "gene": "UniProtKB:O43914",
  "term_id": "GO:0002283",
  "term_label": "neutrophil activation involved in immune response",
  "gene_symbol": "TYROBP"
}